antifungal peptide biosynthetic process [GO:0002783] (biological process) Definition: The chemical reactions and pathways resulting in the formation of an antifungal peptide. Relationships: is a type of antimicrobial peptide biosynthetic process [GO:0002777]; is part of antifungal peptide production [GO:0002781] References: PMID:11807545, PMID:15638771 Sources: GOC:add, ISBN:0781735149 Regulation: RO_0002211 by regulation of antifungal peptide biosynthetic process [GO:0002810]; negatively regulated by GO:0002811; RO_0002213 by GO:0006967